{
  "term_label": "Unknown biological process",
  "gene_name": "IQ domain-containing protein F2",
  "gene_symbol": "IQCF2",
  "term_id": "UNKNOWN:0002",
  "gene": "UniProtKB:Q8IXL9"
}